regulation of secondary cell septum biogenesis [GO:1903395] (biological process) Relationships: is_a regulation of cellular component biogenesis [GO:0044087]; is a type of regulation of mitotic cytokinetic process [GO:1903436]; regulates GO:1990344 References: PMID:23878277 Sources: GOC:TermGenie, GOC:di, GO_REF:0000058 Subtypes: negative regulation of secondary cell septum biogenesis [GO:1903396], positive regulation of secondary cell septum biogenesis [GO:1903397] Definition: Any process that modulates the frequency, rate or extent of secondary cell septum biogenesis.